{
  "term_id": "GO:0005829",
  "gene": "UniProtKB:P48637",
  "term_label": "cytosol",
  "gene_name": "Glutathione synthetase",
  "gene_symbol": "GSS"
}